{
  "gene_name": "UPF0235 protein C15orf40",
  "term_label": "Unknown biological process",
  "gene": "UniProtKB:Q8WUR7",
  "gene_symbol": "C15orf40",
  "term_id": "UNKNOWN:0002"
}